negative regulation of DNA repair [GO:0045738] (biological process) Sources: GOC:go_curators Relationships: is a type of regulation of DNA repair [GO:0006282]; is a type of negative regulation of response to stimulus [GO:0048585]; is a type of negative regulation of DNA metabolic process [GO:0051053]; negatively regulates DNA repair [GO:0006281] Also known as: down regulation of DNA repair, down-regulation of DNA repair, downregulation of DNA repair, inhibition of DNA repair Definition: Any process that stops, prevents, or reduces the frequency, rate or extent of DNA repair. Subtypes: negative regulation of mismatch repair [GO:0032424], GO:1903517, GO:1905052, negative regulation of double-strand break repair [GO:2000780]